{
  "gene_symbol": "HOXB3",
  "term_id": "GO:0005634",
  "term_label": "nucleus",
  "gene_name": "Homeobox protein Hox-B3",
  "gene": "UniProtKB:P14651"
}